{
  "gene": "UniProtKB:Q6XR72",
  "gene_symbol": "SLC30A10",
  "term_label": "zinc ion transmembrane transport",
  "gene_name": "Calcium_manganese antiporter SLC30A10",
  "term_id": "GO:0071577"
}